{
  "gene_name": "Ventral anterior homeobox 2",
  "gene": "UniProtKB:Q9UIW0",
  "term_id": "GO:0007420",
  "term_label": "brain development",
  "gene_symbol": "VAX2"
}